endospore coat [GO:0043593] (cellular component) Definition: The layer in a bacterial endospore that lies under the exosporium, and is impermeable to many toxic molecules. The coat may also contain enzymes that are involved in endospore germination. Relationships: is a type of cellular anatomical structure [GO:0110165]; is part of endospore external encapsulating structure [GO:0043591] Sources: GOC:mlg